{
  "gene_name": "Pro-neuregulin-2, membrane-bound isoform",
  "term_id": "GO:0035556",
  "term_label": "intracellular signal transduction",
  "gene_symbol": "NRG2",
  "gene": "UniProtKB:O14511"
}